malonyl-CoA catabolic process [GO:2001294] (biological process) Sources: GOC:yaf Definition: The chemical reactions and pathways resulting in the breakdown of malonyl-CoA, the S-malonyl derivative of coenzyme A. Relationships: is a type of sulfur compound catabolic process [GO:0044273]; is a type of purine-containing compound catabolic process [GO:0072523]; is a type of nucleoside phosphate catabolic process [GO:1901292]; is a type of malonyl-CoA metabolic process [GO:2001293] Also known as: malonyl-CoA breakdown, malonyl-CoA catabolism, malonyl-CoA degradation